tensidol A biosynthetic process [GO:1900605] (biological process) Sources: GOC:TermGenie, GOC:di Relationships: is a type of ketone biosynthetic process [GO:0042181]; is a type of amide biosynthetic process [GO:0043604]; is a type of secondary metabolite biosynthetic process [GO:0044550] Definition: The chemical reactions and pathways resulting in the formation of tensidol A. Regulation: regulated by regulation of tensidol A biosynthetic process [GO:1900707]; negatively regulated by negative regulation of tensidol A biosynthetic process [GO:1900708]; positively regulated by GO:1900709 Also known as: tensidol A anabolism, tensidol A biosynthesis, tensidol A formation, tensidol A synthesis